{
  "gene": "UniProtKB:Q9HBG6",
  "gene_symbol": "IFT122",
  "term_label": "non-motile cilium assembly",
  "gene_name": "Intraflagellar transport protein 122 homolog",
  "term_id": "GO:1905515"
}